{
  "term_label": "Unknown molecular function",
  "term_id": "UNKNOWN:0001",
  "gene": "UniProtKB:O00471",
  "gene_name": "Exocyst complex component 5",
  "gene_symbol": "EXOC5"
}